clathrin-uncoating ATPase activity [GO:1990833] (molecular function) Definition: Catalysis of the reaction: ATP + H2O = ADP + phosphate. Catalysis of the removal of clathrin from vesicle membranes, coupled to the hydrolysis of ATP. Relationships: is a type of ATP-dependent activity [GO:0140657]; is part of GO:0072318 References: PMID:6146630, PMID:8363588